fever generation [GO:0001660] (biological process) Also known as: pyrexia Definition: The heat generation process that results in a rise in body temperature above the normal, often as a response to infection. Regulation: regulated by GO:0031620; negatively regulated by negative regulation of fever generation [GO:0031621]; positively regulated by positive regulation of fever generation [GO:0031622]; regulated by regulation of fever generation by prostaglandin biosynthetic process [GO:0100008]; regulated by regulation of fever generation by prostaglandin secretion [GO:0100009]; positively regulated by positive regulation of fever generation by prostaglandin biosynthetic process [GO:0100010]; positively regulated by positive regulation of fever generation by prostaglandin secretion [GO:0100011] Sources: GOC:dph, GOC:jl Relationships: is a type of acute-phase response [GO:0006953]; is a type of heat generation [GO:0031649]